{
  "term_id": "GO:0045026",
  "gene": "UniProtKB:A0A1B0GTQ4",
  "gene_name": "Protein myomixer",
  "gene_symbol": "MYMX",
  "term_label": "plasma membrane fusion"
}